(S)-2-hydroxyglutarate dehydrogenase (quinone) activity [GO:0140696] (molecular function) Relationships: is a type of GO:0016901; is a type of (S)-2-hydroxyglutarate dehydrogenase activity [GO:0047545] References: PMID:30498244 Sources: RHEA:58664 Also known as: (S)-2-hydroxyglutarate dehydrogenase activity, L-2-hydroxyglutarate dehydrogenase activity Definition: Catalysis of the reaction: (S)-2-hydroxyglutarate + a quinone = 2-oxoglutarate + a quinol.